{
  "gene_name": "Ubiquitin carboxyl-terminal hydrolase 17-like protein 11",
  "gene": "UniProtKB:C9JVI0",
  "term_label": "regulation of apoptotic process",
  "term_id": "GO:0042981",
  "gene_symbol": "USP17L11"
}